annular furrow extracellular matrix [GO:0060108] (cellular component) Sources: GOC:dph, GOC:kmv, ISSN:15518507 Relationships: is a type of cellular anatomical structure [GO:0110165]; is part of cortical layer of collagen and cuticulin-based cuticle extracellular matrix [GO:0060106] Definition: The extracellular matrix part that is a regularly spaced indentation in the outer cortical layer of the cuticle. The pattern of annular furrows corresponds to sites of invaginations in hypodermal cell membranes that, in turn, correspond to submembranous regions where actin microfilament bundles assemble early in lethargus, the first phase of the molting cycle in which activity and feeding decline.